{
  "gene_symbol": "DKC1",
  "term_label": "rRNA pseudouridine synthesis",
  "term_id": "GO:0031118",
  "gene": "UniProtKB:O60832",
  "gene_name": "H_ACA ribonucleoprotein complex subunit DKC1"
}